{
  "gene_symbol": "EEF1A2",
  "gene": "UniProtKB:Q05639",
  "gene_name": "Elongation factor 1-alpha 2",
  "term_label": "translation",
  "term_id": "GO:0006412"
}